neurotransmitter receptor transport, endosome to postsynaptic membrane [GO:0098887] (biological process) Also known as: postsynaptic neurotransmitter receptor endosomal trafficking Regulation: regulated by GO:0099152 Sources: GOC:dos Relationships: is a type of neurotransmitter receptor transport to postsynaptic membrane [GO:0098969]; is a type of neurotransmitter receptor transport, endosome to plasma membrane [GO:0099639] Definition: The directed movement of neurotransmitter receptor from the postsynaptic endosome to the postsynaptic membrane in transport vesicles.